{
  "term_label": "kainate selective glutamate receptor complex",
  "gene_name": "Glutamate receptor ionotropic, kainate 2",
  "gene_symbol": "GRIK2",
  "gene": "UniProtKB:Q13002",
  "term_id": "GO:0032983"
}